{
  "gene_name": "Putative uncharacterized protein encoded by LINC00469",
  "gene_symbol": "LINC00469",
  "gene": "UniProtKB:Q8N7U9",
  "term_id": "UNKNOWN:0002",
  "term_label": "Unknown biological process"
}